{
  "gene_name": "Tumor necrosis factor ligand superfamily member 15",
  "gene": "UniProtKB:O95150",
  "term_id": "GO:0007166",
  "gene_symbol": "TNFSF15",
  "term_label": "cell surface receptor signaling pathway"
}